{
  "term_label": "superoxide-generating NADPH oxidase activator activity",
  "gene_name": "Neutrophil cytosol factor 4",
  "term_id": "GO:0016176",
  "gene": "UniProtKB:Q15080",
  "gene_symbol": "NCF4"
}